{
  "gene": "UniProtKB:P00749",
  "term_label": "fibrinolysis",
  "gene_name": "Urokinase-type plasminogen activator",
  "gene_symbol": "PLAU",
  "term_id": "GO:0042730"
}